{
  "gene_symbol": "FAM217B",
  "term_label": "Unknown biological process",
  "term_id": "UNKNOWN:0002",
  "gene_name": "Protein FAM217B",
  "gene": "UniProtKB:Q9NTX9"
}